negative regulation of pollen tube guidance [GO:0160068] (biological process) Relationships: is a type of negative regulation of positive chemotaxis [GO:0050928]; negatively regulates pollen tube guidance [GO:0010183] Definition: Any process that decreases the rate, frequency or extent of pollen tube guidance towards ovules. This is one mechanism to prevent polytuby, the simultaneous penetration of ovules by multiple pollen tubes. Also known as: prevention of polytuby References: PMID:33790463